{
  "term_id": "GO:0003714",
  "term_label": "transcription corepressor activity",
  "gene_symbol": "SIN3A",
  "gene_name": "Paired amphipathic helix protein Sin3a",
  "gene": "UniProtKB:Q96ST3"
}